{
  "term_label": "sulfurtransferase activity",
  "gene": "UniProtKB:Q16762",
  "term_id": "GO:0016783",
  "gene_symbol": "TST",
  "gene_name": "Thiosulfate sulfurtransferase"
}